companion cell differentiation [GO:0048758] (biological process) Definition: The process in which a relatively unspecialized cell acquires specialized features of a companion cell. The companion cell is the specialized parenchyma cell associated with a sieve-tube member in angiosperm phloem and arising from the same mother cell as the sieve-tube member. Sources: CL:0000284, GOC:jid Relationships: is a type of plant parenchymal cell differentiation [GO:0048760]; is part of phloem development [GO:0010088]